5-O-phosphono-alpha-D-ribofuranosyl diphosphate binding [GO:1902248] (molecular function) References: PMID:4314233 Sources: GOC:TermGenie, GOC:mah Also known as: 5-phosphoribose 1-diphosphate binding, phosphoribosylpyrophosphate binding Relationships: is a type of anion binding [GO:0043168]; is a type of carbohydrate derivative binding [GO:0097367] Definition: Binding to 5-O-phosphono-alpha-D-ribofuranosyl diphosphate.